{
  "term_label": "spliceosomal snRNP assembly",
  "gene_name": "Gem-associated protein 5",
  "gene": "UniProtKB:Q8TEQ6",
  "gene_symbol": "GEMIN5",
  "term_id": "GO:0000387"
}